{
  "gene_name": "Apoptosis facilitator Bcl-2-like protein 14",
  "term_label": "positive regulation of extrinsic apoptotic signaling pathway",
  "gene": "UniProtKB:Q9BZR8",
  "gene_symbol": "BCL2L14",
  "term_id": "GO:2001238"
}